{
  "term_id": "GO:0047238",
  "term_label": "glucuronosyl-N-acetylgalactosaminyl-proteoglycan 4-beta-N-acetylgalactosaminyltransferase activity",
  "gene_name": "Chondroitin sulfate synthase 1",
  "gene": "UniProtKB:Q86X52",
  "gene_symbol": "CHSY1"
}